{
  "term_label": "DNA-binding transcription factor activity, RNA polymerase II-specific",
  "term_id": "GO:0000981",
  "gene_symbol": "DUXB",
  "gene": "UniProtKB:A0A1W2PPF3",
  "gene_name": "Double homeobox protein B"
}